{
  "gene_name": "Transmembrane emp24 domain-containing protein 7",
  "term_label": "COPII-coated ER to Golgi transport vesicle",
  "gene": "UniProtKB:Q9Y3B3",
  "gene_symbol": "TMED7",
  "term_id": "GO:0030134"
}